{
  "gene": "UniProtKB:Q9H2H8",
  "gene_symbol": "PPIL3",
  "term_id": "GO:0071013",
  "term_label": "catalytic step 2 spliceosome",
  "gene_name": "Peptidyl-prolyl cis-trans isomerase-like 3"
}